positive regulation of macrophage antigen processing and presentation [GO:0002618] (biological process) Definition: Any process that activates or increases the frequency, rate, or extent of macrophage antigen processing and presentation. Also known as: up regulation of macrophage antigen processing and presentation, up-regulation of macrophage antigen processing and presentation, upregulation of macrophage antigen processing and presentation, activation of macrophage antigen processing and presentation, stimulation of macrophage antigen processing and presentation Sources: GOC:add Relationships: is a type of GO:0002579; is a type of regulation of macrophage antigen processing and presentation [GO:0002616]; positively regulates GO:0002472